{
  "gene_symbol": "SMIM10L1",
  "term_id": "UNKNOWN:0003",
  "term_label": "Unknown cellular component",
  "gene_name": "Small integral membrane protein 10-like protein 1",
  "gene": "UniProtKB:P0DMW3"
}